{
  "term_label": "Unknown cellular component",
  "gene": "UniProtKB:Q9H000",
  "gene_name": "E3 ubiquitin-protein ligase makorin-2",
  "term_id": "UNKNOWN:0003",
  "gene_symbol": "MKRN2"
}